{
  "term_label": "myosin filament",
  "term_id": "GO:0032982",
  "gene_name": "Myosin-1",
  "gene": "UniProtKB:P12882",
  "gene_symbol": "MYH1"
}